regulation of eosinophil extravasation [GO:2000419] (biological process) Sources: GOC:mah Definition: Any process that modulates the frequency, rate or extent of eosinophil extravasation. Relationships: is a type of regulation of cellular extravasation [GO:0002691]; is a type of GO:2000416; regulates eosinophil extravasation [GO:0072682] Subtypes: GO:2000420, GO:2000421